{
  "gene": "UniProtKB:O94972",
  "gene_symbol": "TRIM37",
  "term_id": "GO:0051865",
  "term_label": "protein autoubiquitination",
  "gene_name": "E3 ubiquitin-protein ligase TRIM37"
}